{
  "term_id": "GO:0006006",
  "gene_symbol": "DCXR",
  "gene": "UniProtKB:Q7Z4W1",
  "term_label": "glucose metabolic process",
  "gene_name": "L-xylulose reductase"
}